{
  "gene_name": "Augurin",
  "term_label": "regulation of cell population proliferation",
  "gene_symbol": "ECRG4",
  "gene": "UniProtKB:Q9H1Z8",
  "term_id": "GO:0042127"
}